negative regulation of starch catabolic process [GO:2000882] (biological process) Relationships: is_a GO:0009895; is a type of negative regulation of macromolecule metabolic process [GO:0010605]; is a type of negative regulation of carbohydrate metabolic process [GO:0045912]; is_a GO:2000881; negatively regulates starch catabolic process [GO:0005983] Also known as: negative regulation of starch breakdown, negative regulation of starch catabolism, negative regulation of starch degradation Definition: Any process that stops, prevents or reduces the frequency, rate or extent of starch catabolic process. Sources: GOC:obol Subtypes: GO:2000946